{
  "term_label": "protein kinase binding",
  "gene_symbol": "TSKS",
  "gene": "UniProtKB:Q9UJT2",
  "term_id": "GO:0019901",
  "gene_name": "Testis-specific serine kinase substrate"
}